{
  "gene_name": "N-acylneuraminate-9-phosphatase",
  "term_id": "UNKNOWN:0003",
  "gene": "UniProtKB:Q8TBE9",
  "gene_symbol": "NANP",
  "term_label": "Unknown cellular component"
}